{
  "term_label": "Unknown molecular function",
  "gene": "UniProtKB:Q0IIN9",
  "gene_symbol": "ZNF252P-AS1",
  "term_id": "UNKNOWN:0001",
  "gene_name": "Putative uncharacterized protein ZNF252P-AS1"
}